regulation of chitin metabolic process [GO:0032882] (biological process) Definition: Any process that modulates the frequency, rate or extent of the chemical reactions and pathways involving chitin. Sources: GOC:mah Also known as: regulation of chitin metabolism Relationships: is a type of regulation of polysaccharide metabolic process [GO:0032881]; regulates GO:0006030 Subtypes: GO:0032883